{
  "gene_symbol": "RGS21",
  "term_id": "GO:0005096",
  "term_label": "GTPase activator activity",
  "gene_name": "Regulator of G-protein signaling 21",
  "gene": "UniProtKB:Q2M5E4"
}